regulation of cuticle pigmentation [GO:0048079] (biological process) Relationships: is a type of regulation of developmental pigmentation [GO:0048070]; regulates cuticle pigmentation [GO:0048067] Definition: Any process that modulates the frequency, rate or extent of establishment of a pattern of pigment in the cuticle of an organism. Subtypes: GO:0048080, positive regulation of cuticle pigmentation [GO:0048081], regulation of adult chitin-containing cuticle pigmentation [GO:0048082] Sources: GOC:jid